{
  "gene": "UniProtKB:Q9BXP8",
  "term_label": "proteolysis",
  "gene_symbol": "PAPPA2",
  "gene_name": "Pappalysin-2",
  "term_id": "GO:0006508"
}